positive regulation of endoplasmic reticulum calcium ion concentration [GO:0032470] (biological process) Subtypes: positive regulation of smooth endoplasmic reticulum calcium ion concentration [GO:0051564] Also known as: elevation of ER calcium ion concentration, elevation of calcium ion concentration in endoplasmic reticulum, elevation of endoplasmic reticulum calcium ion concentration, endoplasmic reticulum calcium ion concentration elevation Definition: Any process that increases the concentration of calcium ions in the endoplasmic reticulum. Relationships: is a type of GO:0032469 Sources: GOC:mah